{
  "term_label": "Unknown cellular component",
  "term_id": "UNKNOWN:0003",
  "gene_symbol": "SMG8",
  "gene": "UniProtKB:Q8ND04",
  "gene_name": "Nonsense-mediated mRNA decay factor SMG8"
}